{
  "term_label": "translational termination",
  "gene_name": "ATP-binding cassette sub-family E member 1",
  "gene_symbol": "ABCE1",
  "gene": "UniProtKB:P61221",
  "term_id": "GO:0006415"
}